{
  "gene": "UniProtKB:Q9H7C4",
  "term_label": "neuromuscular junction",
  "gene_name": "Syncoilin",
  "gene_symbol": "SYNC",
  "term_id": "GO:0031594"
}